{
  "term_id": "GO:0005634",
  "gene": "UniProtKB:Q13569",
  "gene_symbol": "TDG",
  "term_label": "nucleus",
  "gene_name": "G_T mismatch-specific thymine DNA glycosylase"
}